{
  "gene": "UniProtKB:Q15018",
  "gene_symbol": "ABRAXAS2",
  "term_id": "GO:0090307",
  "gene_name": "BRISC complex subunit Abraxas 2",
  "term_label": "mitotic spindle assembly"
}